{
  "gene_symbol": "ORMDL2",
  "gene": "UniProtKB:Q53FV1",
  "term_label": "intracellular sphingolipid homeostasis",
  "gene_name": "ORM1-like protein 2",
  "term_id": "GO:0090156"
}